{
  "term_id": "GO:0048666",
  "gene": "UniProtKB:Q96QS3",
  "term_label": "neuron development",
  "gene_symbol": "ARX",
  "gene_name": "Homeobox protein ARX"
}